L-dopa decarboxylase activator activity [GO:0036478] (molecular function) Also known as: DDC activator activity Sources: GOC:PARL, GOC:bf Note: GO:0036478 is reserved for cases when the activator directly interacts with L-dopa decarboxylase. When activation of L-dopa decarboxylase activity is achieved without enzyme binding, or when the mechanism of regulation is unknown, instead annotate to 'positive regulation of L-dopa decarboxylase activity ; GO:1903200'. Definition: Interacts with and increases L-dopa decarboxylase activity. Relationships: is a type of enzyme activator activity [GO:0008047]; positively regulates L-dopa decarboxylase activity [GO:0036468]